{
  "gene_symbol": "TNF",
  "term_label": "positive regulation of canonical NF-kappaB signal transduction",
  "gene": "UniProtKB:P01375",
  "term_id": "GO:0043123",
  "gene_name": "Tumor necrosis factor"
}